{
  "gene_name": "Brain-specific angiogenesis inhibitor 1-associated protein 2-like protein 1",
  "gene": "UniProtKB:Q9UHR4",
  "term_label": "nucleoplasm",
  "gene_symbol": "BAIAP2L1",
  "term_id": "GO:0005654"
}